{
  "gene_symbol": "OR14J1",
  "gene_name": "Olfactory receptor 14J1",
  "gene": "UniProtKB:Q9UGF5",
  "term_id": "UNKNOWN:0002",
  "term_label": "Unknown biological process"
}